{
  "term_id": "GO:0031490",
  "gene_name": "Lysine-specific demethylase 6A",
  "term_label": "chromatin DNA binding",
  "gene_symbol": "KDM6A",
  "gene": "UniProtKB:O15550"
}